{
  "gene": "UniProtKB:Q96CW1",
  "term_label": "AP-1 adaptor complex",
  "term_id": "GO:0030121",
  "gene_name": "AP-2 complex subunit mu",
  "gene_symbol": "AP2M1"
}